{
  "gene_symbol": "RNASE12",
  "term_label": "Unknown molecular function",
  "term_id": "UNKNOWN:0001",
  "gene": "UniProtKB:Q5GAN4",
  "gene_name": "Probable inactive ribonuclease-like protein 12"
}